positive regulation of chromosome organization [GO:2001252] (biological process) Subtypes: positive regulation of telomere maintenance [GO:0032206], positive regulation of sister chromatid cohesion [GO:0045876], positive regulation of mitotic sister chromatid segregation [GO:0062033], positive regulation of oocyte karyosome formation [GO:0120315], positive regulation of synaptonemal complex assembly [GO:1905088], positive regulation of chromatin organization [GO:1905269], GO:1905561, positive regulation of chromosome condensation [GO:1905821] Definition: Any process that activates or increases the frequency, rate or extent of chromosome organization. Relationships: is a type of GO:0010638; is a type of regulation of chromosome organization [GO:0033044]; positively regulates chromosome organization [GO:0051276] Sources: GOC:obol Also known as: positive regulation of chromosome organisation, positive regulation of chromosome organization and biogenesis, positive regulation of maintenance of genome integrity, positive regulation of nuclear genome maintenance